{
  "term_label": "Unknown biological process",
  "gene_name": "Uncharacterized protein",
  "term_id": "UNKNOWN:0002",
  "gene_symbol": "LOC728392",
  "gene": "UniProtKB:A0A494C1I1"
}